positive regulation of tooth mineralization [GO:0070172] (biological process) Definition: Any process that activates or increases the frequency, rate or extent of tooth mineralization, the deposition of calcium salts in tooth structures. Sources: GOC:BHF, GOC:mah Relationships: is a type of positive regulation of biomineral tissue development [GO:0070169]; is a type of regulation of tooth mineralization [GO:0070170]; positively regulates tooth mineralization [GO:0034505] Subtypes: positive regulation of enamel mineralization [GO:0070175]